{
  "term_id": "GO:0005829",
  "gene_name": "Microtubule-associated protein 1B",
  "gene_symbol": "MAP1B",
  "gene": "UniProtKB:P46821",
  "term_label": "cytosol"
}